activated T cell autonomous cell death [GO:0070238] (biological process) Also known as: ACAD, activated T cell apoptosis, activated cell autonomous cell death, activated T lymphocyte autonomous cell death, activated T-cell autonomous cell death, activated T-lymphocyte autonomous cell death Sources: GOC:add, GOC:mtg_apoptosis, ISBN:0781765196 Relationships: is a type of GO:0070231; is part of T cell homeostasis [GO:0043029] Regulation: regulated by GO:0070239; negatively regulated by negative regulation of activated T cell autonomous cell death [GO:0070240]; positively regulated by GO:0070241 Definition: A T cell apoptotic process that occurs towards the end of the expansion phase following the initial activation of mature T cells by antigen via the accumulation of pro-apoptotic gene products and decrease in anti-apoptotic gene products.